{
  "gene_symbol": "OR2B2",
  "gene_name": "Olfactory receptor 2B2",
  "term_label": "olfactory receptor activity",
  "term_id": "GO:0004984",
  "gene": "UniProtKB:Q9GZK3"
}